{
  "gene_symbol": "MS4A15",
  "gene_name": "Membrane-spanning 4-domains subfamily A member 15",
  "term_id": "GO:0007166",
  "term_label": "cell surface receptor signaling pathway",
  "gene": "UniProtKB:Q8N5U1"
}